{
  "gene_name": "Activator of apoptosis harakiri",
  "term_label": "positive regulation of apoptotic process",
  "term_id": "GO:0043065",
  "gene": "UniProtKB:O00198",
  "gene_symbol": "HRK"
}